{
  "gene": "UniProtKB:P40763",
  "gene_symbol": "STAT3",
  "gene_name": "Signal transducer and activator of transcription 3",
  "term_label": "regulation of transcription by RNA polymerase II",
  "term_id": "GO:0006357"
}